{
  "gene_symbol": "PLPPR4",
  "gene": "UniProtKB:Q7Z2D5",
  "gene_name": "Phospholipid phosphatase-related protein type 4",
  "term_label": "axonogenesis",
  "term_id": "GO:0007409"
}